regulation of postsynaptic density organization [GO:1905874] (biological process) References: PMID:21887379 Sources: GOC:TermGenie, GO_REF:0000058 Relationships: is a type of regulation of organelle organization [GO:0033043]; is a type of regulation of postsynapse organization [GO:0099175]; regulates postsynaptic density organization [GO:0097106] Subtypes: GO:0099151, regulation of postsynaptic density protein 95 clustering [GO:1902897], GO:1905875, positive regulation of postsynaptic density organization [GO:1905876] Also known as: regulation of PSD organization, regulation of post synaptic density organization, regulation of post-synaptic density organization, regulation of postsynaptic density organisation Definition: Any process that modulates the frequency, rate or extent of postsynaptic density organization.